{
  "gene": "UniProtKB:H3BQB6",
  "term_label": "microtubule depolymerization",
  "term_id": "GO:0007019",
  "gene_symbol": "STMND1",
  "gene_name": "Stathmin domain-containing protein 1"
}